regulation of fibroblast migration [GO:0010762] (BP) Sources: GOC:dph, GOC:tb Definition: Any process that modulates the rate, frequency or extent of fibroblast cell migration. Fibroblast cell migration is accomplished by extension and retraction of a pseudopodium. Subtypes: positive regulation of fibroblast migration [GO:0010763], GO:0010764, regulation of hepatic stellate cell migration [GO:0061869] Relationships: is a type of GO:0030334; regulates GO:0010761 Also known as: regulation of fibroblast cell migration